pancreas development [GO:0031016] (biological process) Sources: GOC:cvs Relationships: is a type of animal organ development [GO:0048513] Definition: The process whose specific outcome is the progression of the pancreas over time, from its formation to the mature structure. The pancreas is an endoderm derived structure that produces precursors of digestive enzymes and blood glucose regulating hormones.